response to nitrate [GO:0010167] (biological process) Relationships: is a type of response to nitrogen compound [GO:1901698]; is a type of response to oxygen-containing compound [GO:1901700] Sources: GOC:sm Definition: Any process that results in a change in state or activity of a cell or an organism (in terms of movement, secretion, enzyme production, gene expression, etc.) as a result of a nitrate stimulus. Subtypes: cellular response to nitrate [GO:0071249]